{
  "term_label": "plasma membrane",
  "term_id": "GO:0005886",
  "gene_symbol": "LMBR1L",
  "gene_name": "Protein LMBR1L",
  "gene": "UniProtKB:Q6UX01"
}